{
  "term_id": "GO:0005634",
  "gene_name": "RNA-binding motif, single-stranded-interacting protein 2",
  "term_label": "nucleus",
  "gene_symbol": "RBMS2",
  "gene": "UniProtKB:Q15434"
}